chemorepulsion involved in postnatal olfactory bulb interneuron migration [GO:0021836] (biological process) Also known as: negative chemotaxis involved in postnatal olfactory bulb interneuron migration Definition: The creation and reception of signals that repel olfactory bulb interneurons from the subventricular zone as a component process in tangential migration. Relationships: is a type of negative chemotaxis [GO:0050919]; is part of postnatal olfactory bulb interneuron migration [GO:0021827] References: PMID:12626695 Sources: GOC:cls, GOC:dgh, GOC:dph, GOC:jid, GO_REF:0000021